{
  "gene": "UniProtKB:P52737",
  "gene_name": "Zinc finger protein 136",
  "term_id": "GO:0000978",
  "gene_symbol": "ZNF136",
  "term_label": "RNA polymerase II cis-regulatory region sequence-specific DNA binding"
}